mitochondrial magnesium ion transmembrane transport [GO:0045016] (biological process) Definition: The process in which a magnesium ion (Mg2+) is transported across a mitochondrial membrane, into or out of the mitochondrion. Relationships: is a type of magnesium ion transmembrane transport [GO:1903830] Also known as: mitochondrial magnesium ion transport References: PMID:11254124 Sources: GOC:ai Subtypes: GO:1990616